ent-copalyl diphosphate synthase activity [GO:0009905] (molecular function) Relationships: is a type of GO:0016872 Definition: Catalysis of the reaction: all-trans-geranylgeranyl diphosphate = ent-copalyl diphosphate. Also known as: diterpene cyclase activity, ent-kaurene synthase A activity, ent-kaurene synthetase A activity, ent-copalyl-diphosphate lyase (decyclizing) Sources: EC:5.5.1.13, RHEA:14841